{
  "term_label": "intrinsic apoptotic signaling pathway in response to DNA damage by p53 class mediator",
  "term_id": "GO:0042771",
  "gene": "UniProtKB:O15350",
  "gene_name": "Tumor protein p73",
  "gene_symbol": "TP73"
}